advanced glycation end-product receptor activity [GO:0050785] (molecular function) References: PMID:12453678, PMID:12707408, PMID:7592757, PMID:9224812 Sources: GOC:signaling, Wikipedia:RAGE_(receptor) Also known as: AGE receptor activity, RAGE activity Relationships: is a type of signaling receptor activity [GO:0038023] Definition: Combining with advanced glycation end-products and transmitting the signal to initiate a change in cell activity. Advanced glycation end-products (AGEs) form from a series of chemical reactions after an initial glycation event (a non-enzymatic reaction between reducing sugars and free amino groups of proteins).